{
  "term_label": "beta-catenin binding",
  "gene_name": "Cadherin-9",
  "gene": "UniProtKB:Q9ULB4",
  "term_id": "GO:0008013",
  "gene_symbol": "CDH9"
}